{
  "term_id": "UNKNOWN:0001",
  "gene_name": "Probable G-protein coupled receptor 158",
  "gene_symbol": "GPR158",
  "gene": "UniProtKB:Q5T848",
  "term_label": "Unknown molecular function"
}